{
  "gene_symbol": "PNMA8A",
  "term_label": "Unknown molecular function",
  "gene_name": "Paraneoplastic antigen-like protein 8A",
  "gene": "UniProtKB:Q86V59",
  "term_id": "UNKNOWN:0001"
}